{
  "term_id": "GO:0004558",
  "gene": "UniProtKB:Q2M2H8",
  "gene_name": "Probable maltase-glucoamylase 2",
  "term_label": "alpha-1,4-glucosidase activity",
  "gene_symbol": "MGAM2"
}